palmitoyl hydrolase activity [GO:0098599] (molecular function) Definition: Catalysis of a hydrolase reaction that removes a palmitoyl moiety from some substrate. Relationships: is a type of hydrolase activity [GO:0016787]; is part of macromolecule depalmitoylation [GO:0098734] Sources: GOC:dos, GOC:pg Subtypes: palmitoyl-(protein) hydrolase activity [GO:0008474]